negative regulation of mesenchymal stem cell proliferation [GO:1902461] (biological process) Relationships: is a type of regulation of mesenchymal stem cell proliferation [GO:1902460]; is a type of negative regulation of stem cell proliferation [GO:2000647]; negatively regulates mesenchymal stem cell proliferation [GO:0097168] Definition: Any process that stops, prevents or reduces the frequency, rate or extent of mesenchymal stem cell proliferation. Also known as: down regulation of MSC proliferation, down regulation of mesenchymal stem cell proliferation, down-regulation of MSC proliferation, down-regulation of mesenchymal stem cell proliferation, downregulation of MSC proliferation, downregulation of mesenchymal stem cell proliferation, negative regulation of MSC proliferation, inhibition of MSC proliferation, inhibition of mesenchymal stem cell proliferation References: PMID:18672106 Sources: GOC:TermGenie, GOC:pm